{
  "gene_name": "Monocarboxylate transporter 11",
  "gene_symbol": "SLC16A11",
  "term_label": "Unknown biological process",
  "term_id": "UNKNOWN:0002",
  "gene": "UniProtKB:Q8NCK7"
}